{
  "term_label": "synaptic vesicle membrane",
  "gene": "UniProtKB:O95473",
  "term_id": "GO:0030672",
  "gene_name": "Synaptogyrin-4",
  "gene_symbol": "SYNGR4"
}